{
  "gene_name": "Histidine-rich carboxyl terminus protein 1",
  "gene": "UniProtKB:Q6UXD1",
  "term_id": "UNKNOWN:0002",
  "term_label": "Unknown biological process",
  "gene_symbol": "HRCT1"
}